{
  "term_id": "GO:0042273",
  "gene": "UniProtKB:P61254",
  "term_label": "ribosomal large subunit biogenesis",
  "gene_symbol": "RPL26",
  "gene_name": "Large ribosomal subunit protein uL24"
}